O-succinyltransferase activity [GO:0016750] (molecular function) Sources: GOC:ai Relationships: is a type of O-acyltransferase activity [GO:0008374]; is a type of succinyltransferase activity [GO:0016748] Definition: Catalysis of the transfer of a succinyl group to an oxygen atom on the acceptor molecule. Subtypes: homoserine O-succinyltransferase activity [GO:0008899], GO:0160210